{
  "term_label": "cytoplasm",
  "gene": "UniProtKB:P50616",
  "gene_symbol": "TOB1",
  "gene_name": "Protein Tob1",
  "term_id": "GO:0005737"
}